nucleoplasmic THO complex [GO:0000446] (cellular component) Relationships: is a type of THO complex [GO:0000347]; is a type of transcription elongation factor complex [GO:0008023] Definition: The THO complex when it is acting as a nuclear complex that is required for transcription elongation through genes containing tandemly repeated DNA sequences. In S. cerevisiae, it is composed of four subunits: Hpr1, Tho2, Thp2, and Mft1, while the human complex is composed of 7 subunits. References: PMID:11060033, PMID:11979277, PMID:16983072 Sources: GOC:krc, GOC:se